guanine deglycation [GO:0106044] (biological process) References: PMID:28596309 Relationships: is a type of nucleotide metabolic process [GO:0009117] Subtypes: guanine deglycation, methylglyoxal removal [GO:0106045], guanine deglycation, glyoxal removal [GO:0106046] Definition: The removal of a sugar or dicarbonyl from a glycated guanine.